limb bud formation [GO:0060174] (biological process) Sources: GOC:dgh, GOC:dph Relationships: is a type of anatomical structure formation involved in morphogenesis [GO:0048646]; is part of limb morphogenesis [GO:0035108] Definition: The process pertaining to the initial formation of a limb bud from unspecified parts. This process begins with the formation of a local condensation of mesenchyme cells within the prospective limb field, and ends when a limb bud is recognizable. Also known as: limb formation, limbbud formation